{
  "term_id": "UNKNOWN:0003",
  "term_label": "Unknown cellular component",
  "gene_name": "Mitochondrial adenyl nucleotide antiporter SLC25A24",
  "gene_symbol": "SLC25A24",
  "gene": "UniProtKB:Q6NUK1"
}